{
  "gene_symbol": "PKIA",
  "term_id": "GO:0004862",
  "gene": "UniProtKB:P61925",
  "term_label": "cAMP-dependent protein kinase inhibitor activity",
  "gene_name": "cAMP-dependent protein kinase inhibitor alpha"
}